{
  "term_label": "Unknown biological process",
  "gene": "UniProtKB:Q5T440",
  "term_id": "UNKNOWN:0002",
  "gene_name": "Putative transferase CAF17, mitochondrial",
  "gene_symbol": "IBA57"
}